pyrimidine ribonucleoside metabolic process [GO:0046131] (biological process) Relationships: is a type of GO:0006213; is a type of ribonucleoside metabolic process [GO:0009119] Sources: GOC:ai Subtypes: cytidine metabolic process [GO:0046087], GO:0046108, pyrimidine ribonucleoside biosynthetic process [GO:0046132], GO:0046133 Also known as: pyrimidine ribonucleoside metabolism Definition: The chemical reactions and pathways involving any ribonucleoside, a nucleoside in which pyrimidine base is linked to a ribose (beta-D-ribofuranose) molecule.